{
  "gene_symbol": "MAPK10",
  "term_label": "JNK cascade",
  "gene_name": "Mitogen-activated protein kinase 10",
  "gene": "UniProtKB:P53779",
  "term_id": "GO:0007254"
}